{
  "gene": "UniProtKB:Q96MH2",
  "term_id": "GO:0005654",
  "term_label": "nucleoplasm",
  "gene_symbol": "HEXIM2",
  "gene_name": "Protein HEXIM2"
}